{
  "term_id": "GO:0005737",
  "gene_symbol": "PRKAG3",
  "term_label": "cytoplasm",
  "gene_name": "5'-AMP-activated protein kinase subunit gamma-3",
  "gene": "UniProtKB:Q9UGI9"
}